peptidyl-lysine acetylation [GO:0018394] (biological process) Subtypes: N-terminal peptidyl-lysine acetylation [GO:0018076], internal peptidyl-lysine acetylation [GO:0018393] Sources: GOC:mah Regulation: regulated by GO:2000756; negatively regulated by GO:2000757; positively regulated by GO:2000758 Relationships: is a type of protein acetylation [GO:0006473]; is a type of peptidyl-lysine modification [GO:0018205] Definition: The acetylation of peptidyl-lysine.